negative regulation of metanephric glomerulus development [GO:0072299] (biological process) Relationships: is_a negative regulation of metanephros development [GO:0072217]; is a type of GO:0072298; is a type of negative regulation of glomerulus development [GO:0090194]; negatively regulates metanephric glomerulus development [GO:0072224] Definition: Any process that decreases the rate, frequency or extent of metanephric glomerulus development, the progression of the metanephric glomerulus over time from its initial formation until its mature state. The metanephric glomerulus is a capillary tuft surrounded by Bowman's capsule in nephrons of the vertebrate kidney, or metanephros. Sources: GOC:mtg_kidney_jan10